{
  "gene_name": "Sarcospan",
  "gene": "UniProtKB:Q14714",
  "term_label": "Unknown molecular function",
  "term_id": "UNKNOWN:0001",
  "gene_symbol": "SSPN"
}